{
  "gene_symbol": "TMEM60",
  "term_label": "Unknown cellular component",
  "gene_name": "Transmembrane protein 60",
  "term_id": "UNKNOWN:0003",
  "gene": "UniProtKB:Q9H2L4"
}